cellular senescence [GO:0090398] (biological process) Relationships: is a type of GO:0009987; is part of cellular response to stress [GO:0033554] Regulation: regulated by GO:2000772; negatively regulated by GO:2000773; positively regulated by GO:2000774 Subtypes: stress-induced premature senescence [GO:0090400], oncogene-induced cell senescence [GO:0090402] Definition: A cell aging process stimulated in response to cellular stress, whereby normal cells lose the ability to divide through irreversible cell cycle arrest. References: PMID:28682291 Sources: GOC:BHF